{
  "gene_symbol": "ARHGAP25",
  "gene": "UniProtKB:P42331",
  "gene_name": "Rho GTPase-activating protein 25",
  "term_label": "phagocytosis, engulfment",
  "term_id": "GO:0006911"
}